{
  "gene_symbol": "LPP",
  "gene": "UniProtKB:Q93052",
  "gene_name": "Lipoma-preferred partner",
  "term_id": "GO:0001725",
  "term_label": "stress fiber"
}